{
  "gene": "UniProtKB:Q6UUV9",
  "gene_name": "CREB-regulated transcription coactivator 1",
  "term_label": "nucleus",
  "term_id": "GO:0005634",
  "gene_symbol": "CRTC1"
}